3-alpha-hydroxysteroid 3-dehydrogenase [NAD(P)+] activity [GO:0140169] (molecular function) Note: Note that EC distinguishes stereospecific reactions: EC:1.1.1.213 and EC:1.1.1.50. These are out of scope for GO. Relationships: is a type of steroid dehydrogenase activity, acting on the CH-OH group of donors, NAD or NADP as acceptor [GO:0033764] Definition: Catalysis of the reaction: a 3alpha-hydroxysteroid + NAD(P)+ = a 3-oxosteroid + NAD(P)H + H+. Sources: EC:1.1.1.357